{
  "term_label": "Unknown cellular component",
  "gene": "UniProtKB:Q9HBI6",
  "term_id": "UNKNOWN:0003",
  "gene_symbol": "CYP4F11",
  "gene_name": "Cytochrome P450 4F11"
}